{
  "gene": "UniProtKB:A2RTY3",
  "term_label": "Unknown cellular component",
  "gene_name": "Protein HEATR9",
  "gene_symbol": "HEATR9",
  "term_id": "UNKNOWN:0003"
}